lncRNA processing [GO:0180035] (biological process) Subtypes: co-transcriptional lncRNA 3' end processing, cleavage and polyadenylation pathway [GO:0180034] Definition: Any process involved in the conversion of one or more primary lncRNA transcripts into one or more mature lncRNA molecules. Relationships: is a type of GO:0006396 References: PMID:31276588